{
  "gene_symbol": "ZNF764",
  "term_id": "GO:0000981",
  "term_label": "DNA-binding transcription factor activity, RNA polymerase II-specific",
  "gene": "UniProtKB:Q96H86",
  "gene_name": "Zinc finger protein 764"
}